{
  "gene_symbol": "AHCYL2",
  "term_id": "GO:0005829",
  "gene_name": "Adenosylhomocysteinase 3",
  "gene": "UniProtKB:Q96HN2",
  "term_label": "cytosol"
}